{
  "term_label": "Unknown biological process",
  "gene_name": "LIM and SH3 domain protein 1",
  "gene_symbol": "LASP1",
  "gene": "UniProtKB:Q14847",
  "term_id": "UNKNOWN:0002"
}